{
  "gene_name": "Desmoplakin",
  "gene": "UniProtKB:P15924",
  "term_label": "plasma membrane",
  "gene_symbol": "DSP",
  "term_id": "GO:0005886"
}